cis-Golgi network membrane [GO:0033106] (cellular component) Definition: The lipid bilayer surrounding any of the compartments that make up the cis-Golgi network. Sources: GOC:mah Also known as: cis Golgi network membrane, Golgi cis face membrane Relationships: is a type of bounding membrane of organelle [GO:0098588]; is part of cis-Golgi network [GO:0005801]